{
  "term_id": "GO:0031429",
  "gene": "UniProtKB:Q9NX24",
  "gene_symbol": "NHP2",
  "gene_name": "H_ACA ribonucleoprotein complex subunit 2",
  "term_label": "box H/ACA snoRNP complex"
}